negative regulation of interleukin-33 production [GO:0150128] (biological process) Also known as: negative regulation of interleukin-33 biosynthetic process, negative regulation of interleukin-33 secretion References: PMID:29778524 Sources: GOC:aruk Definition: Any process that stops, prevents or reduces the frequency, rate or extent of interleukin-33 production. Relationships: is a type of negative regulation of cytokine production [GO:0001818]; is a type of regulation of interleukin-33 production [GO:0150127]; negatively regulates GO:0072639